{
  "gene_name": "ADP-ribosylation factor 3",
  "gene": "UniProtKB:P61204",
  "term_label": "plasma membrane",
  "gene_symbol": "ARF3",
  "term_id": "GO:0005886"
}